{
  "gene_symbol": "CRLF2",
  "gene_name": "Cytokine receptor-like factor 2",
  "term_id": "GO:0009897",
  "term_label": "external side of plasma membrane",
  "gene": "UniProtKB:Q9HC73"
}